haustorium neck formation [GO:0075197] (biological process) Definition: The assembly by the symbiont of a neck-like structure for the purpose of penetration into its host organism. The neck-like structure connects haustorium mother cell and haustorium. The host is defined as the larger of the organisms involved in a symbiotic interaction. Sources: GOC:pamgo_curators, Wikipedia:Haustorium Also known as: formation of symbiont haustorium neck for entry into host, symbiont haustorium neck formation for entry into host Note: Note that this term should not be used to annotate gene products of the host. It should only be used to annotate those gene products from the symbiont involved in this process. Relationships: is a type of GO:0075015 Regulation: regulated by modulation of symbiont haustorium neck formation for entry into host [GO:0075198]; positively regulated by positive regulation of symbiont haustorium neck formation for entry into host [GO:0075199]